{
  "term_id": "GO:0015631",
  "term_label": "tubulin binding",
  "gene": "UniProtKB:Q8WYA0",
  "gene_symbol": "IFT81",
  "gene_name": "Intraflagellar transport protein 81 homolog"
}